{
  "gene": "UniProtKB:Q01813",
  "gene_symbol": "PFKP",
  "term_id": "GO:0061621",
  "gene_name": "ATP-dependent 6-phosphofructokinase, platelet type",
  "term_label": "canonical glycolysis"
}